{
  "gene_symbol": "SMIM42",
  "term_label": "Unknown cellular component",
  "gene": "UniProtKB:A0A5F9ZH02",
  "term_id": "UNKNOWN:0003",
  "gene_name": "Small integral membrane protein 42"
}